{
  "gene_name": "F-box only protein 9",
  "gene": "UniProtKB:Q9UK97",
  "term_label": "ubiquitin-like ligase-substrate adaptor activity",
  "term_id": "GO:1990756",
  "gene_symbol": "FBXO9"
}